{
  "gene_name": "Noelin-2",
  "term_id": "GO:0005615",
  "term_label": "extracellular space",
  "gene_symbol": "OLFM2",
  "gene": "UniProtKB:O95897"
}